{
  "gene": "UniProtKB:Q13568",
  "term_label": "regulation of transcription by RNA polymerase II",
  "gene_name": "Interferon regulatory factor 5",
  "gene_symbol": "IRF5",
  "term_id": "GO:0006357"
}